fructose-6-phosphate phosphoketolase activity [GO:0047905] (MF) Definition: Catalysis of the reaction: D-fructose 6-phosphate + phosphate = acetyl phosphate + D-erythrose 4-phosphate + H2O. Also known as: D-fructose-6-phosphate D-erythrose-4-phosphate-lyase (adding phosphate; acetyl-phosphate-forming), D-fructose-6-phosphate D-erythrose-4-phosphate-lyase (phosphate-acetylating) activity Relationships: is_a aldehyde-lyase activity [GO:0016832] Sources: EC:4.1.2.22, MetaCyc:FRUCTOSE-6-PHOSPHATE-PHOSPHOKETOLASE-RXN